{
  "term_id": "GO:0004714",
  "gene_symbol": "TIE1",
  "term_label": "transmembrane receptor protein tyrosine kinase activity",
  "gene": "UniProtKB:P35590",
  "gene_name": "Tyrosine-protein kinase receptor Tie-1"
}